{
  "gene": "UniProtKB:Q9UGJ0",
  "term_label": "protein kinase regulator activity",
  "gene_name": "5'-AMP-activated protein kinase subunit gamma-2",
  "term_id": "GO:0019887",
  "gene_symbol": "PRKAG2"
}